{
  "gene_symbol": "ARHGEF4",
  "gene_name": "Rho guanine nucleotide exchange factor 4",
  "gene": "UniProtKB:Q9NR80",
  "term_id": "GO:0005085",
  "term_label": "guanyl-nucleotide exchange factor activity"
}